{
  "gene_symbol": "COIL",
  "term_id": "GO:0030619",
  "gene_name": "Coilin",
  "term_label": "U1 snRNA binding",
  "gene": "UniProtKB:P38432"
}